{
  "gene_symbol": "APLNR",
  "gene_name": "Apelin receptor",
  "gene": "UniProtKB:P35414",
  "term_id": "GO:0007507",
  "term_label": "heart development"
}